{
  "term_id": "GO:0007268",
  "gene_symbol": "NPY5R",
  "term_label": "chemical synaptic transmission",
  "gene_name": "Neuropeptide Y receptor type 5",
  "gene": "UniProtKB:Q15761"
}